{
  "gene": "UniProtKB:Q6YFQ2",
  "term_id": "UNKNOWN:0002",
  "term_label": "Unknown biological process",
  "gene_symbol": "COX6B2",
  "gene_name": "Cytochrome c oxidase subunit 6B2"
}